{
  "gene_symbol": "E4F1",
  "term_id": "GO:0000978",
  "gene_name": "Transcription factor E4F1",
  "gene": "UniProtKB:Q66K89",
  "term_label": "RNA polymerase II cis-regulatory region sequence-specific DNA binding"
}